{
  "term_id": "GO:0050807",
  "term_label": "regulation of synapse organization",
  "gene_symbol": "CAMK1",
  "gene_name": "Calcium_calmodulin-dependent protein kinase type 1",
  "gene": "UniProtKB:Q14012"
}